cell-abiotic substrate adhesion [GO:0036164] (biological process) Relationships: is a type of GO:0031589 Definition: The attachment of a cell to an underlying abiotic (non-living) substrate via adhesion molecules. Sources: GOC:di Also known as: cell-abiotic surface adhesion